{
  "term_id": "GO:0030215",
  "gene_symbol": "SEMA4D",
  "gene": "UniProtKB:Q92854",
  "term_label": "semaphorin receptor binding",
  "gene_name": "Semaphorin-4D"
}